volume-sensitive anion channel activity [GO:0005225] (MF) Definition: Enables the transmembrane transfer of a monoatomic anion by a volume-sensitive channel. A volume-sensitive channel is a channel that responds to changes in the volume of a cell. Sources: GOC:dph, GOC:tb Also known as: volume-regulated channel Relationships: is a type of monoatomic anion channel activity [GO:0005253] Subtypes: volume-sensitive chloride channel activity [GO:0072320]